{
  "term_id": "GO:0004930",
  "term_label": "G protein-coupled receptor activity",
  "gene": "UniProtKB:Q5T6X5",
  "gene_symbol": "GPRC6A",
  "gene_name": "G-protein coupled receptor family C group 6 member A"
}